{
  "term_id": "UNKNOWN:0003",
  "term_label": "Unknown cellular component",
  "gene_symbol": "ARRDC1-AS1",
  "gene": "UniProtKB:Q9H2J1",
  "gene_name": "Uncharacterized protein ARRDC1-AS1"
}